{
  "gene_name": "Acyl carrier protein, mitochondrial",
  "term_label": "respiratory chain complex I",
  "gene": "UniProtKB:O14561",
  "gene_symbol": "NDUFAB1",
  "term_id": "GO:0045271"
}